bacterial-type flagellum assembly [GO:0044780] (biological process) Also known as: bacterial flagellum assembly Relationships: is a type of cell projection assembly [GO:0030031]; is a type of GO:0044781; is a type of membraneless organelle assembly [GO:0140694] Regulation: regulated by GO:1902208; negatively regulated by negative regulation of bacterial-type flagellum assembly [GO:1902209]; positively regulated by positive regulation of bacterial-type flagellum assembly [GO:1902210] Sources: GOC:jl Definition: The assembly of a bacterial-type flagellum, a motor complex composed of an extracellular helical protein filament coupled to a rotary motor embedded in the cell envelope which functions in cell motility.